{
  "gene_symbol": "AXIN2",
  "gene": "UniProtKB:Q9Y2T1",
  "term_id": "GO:0031625",
  "term_label": "ubiquitin protein ligase binding",
  "gene_name": "Axin-2"
}